{
  "gene_name": "Uncharacterized protein KIAA1958",
  "term_id": "UNKNOWN:0002",
  "gene_symbol": "KIAA1958",
  "term_label": "Unknown biological process",
  "gene": "UniProtKB:Q8N8K9"
}